{
  "term_id": "UNKNOWN:0002",
  "term_label": "Unknown biological process",
  "gene_symbol": "CSMD3",
  "gene_name": "CUB and sushi domain-containing protein 3",
  "gene": "UniProtKB:Q7Z407"
}